{
  "gene_symbol": "AMER3",
  "gene_name": "APC membrane recruitment protein 3",
  "gene": "UniProtKB:Q8N944",
  "term_label": "beta-catenin binding",
  "term_id": "GO:0008013"
}